helper T cell diapedesis [GO:0035685] (biological process) Also known as: T-helper cell diapedesis, helper T-cell diapedesis Relationships: is a type of diapedesis [GO:0050904]; is a type of GO:0072678; is part of helper T cell extravasation [GO:0035684] Sources: CL:0000912, GOC:BHF Definition: The passage of a helper T cell between the tight junctions of endothelial cells lining blood vessels, typically the fourth and final step of cellular extravasation. Subtypes: T-helper 1 cell diapedesis [GO:0035688]